inositol catabolic process [GO:0019310] (biological process) Relationships: is a type of inositol metabolic process [GO:0006020]; is a type of polyol catabolic process [GO:0046174] Sources: GOC:go_curators Definition: The chemical reactions and pathways resulting in the breakdown of inositol, 1,2,3,4,5,6-cyclohexanehexol, a growth factor for animals and microorganisms. Also known as: inositol breakdown, inositol catabolism, inositol degradation, vitamin Bh catabolic process, vitamin Bh catabolism, myo-inositol catabolic process, myo-inositol catabolism